{
  "gene": "UniProtKB:Q15270",
  "gene_name": "NK1 transcription factor-related protein 1",
  "gene_symbol": "NKX1-1",
  "term_label": "DNA-binding transcription factor activity, RNA polymerase II-specific",
  "term_id": "GO:0000981"
}